negative regulation of acetate catabolic process [GO:0045753] (biological process) Sources: GOC:go_curators Also known as: down regulation of acetate catabolic process, down-regulation of acetate catabolic process, downregulation of acetate catabolic process, negative regulation of acetate breakdown, negative regulation of acetate catabolism, negative regulation of acetate degradation, inhibition of acetate catabolic process Relationships: is a type of negative regulation of catabolic process [GO:0009895]; is a type of GO:0045734; is a type of negative regulation of small molecule metabolic process [GO:0062014]; negatively regulates acetate catabolic process [GO:0045733] Definition: Any process that stops, prevents, or reduces the frequency, rate or extent of the chemical reactions and pathways resulting in the breakdown of acetate.